{
  "term_label": "cellular response to heat",
  "gene_name": "DnaJ homolog subfamily A member 4",
  "term_id": "GO:0034605",
  "gene": "UniProtKB:Q8WW22",
  "gene_symbol": "DNAJA4"
}